negative regulation of inward rectifier potassium channel activity [GO:1903609] (biological process) Definition: Any process that stops, prevents or reduces the frequency, rate or extent of inward rectifier potassium channel activity. References: PMID:18923542 Sources: GOC:BHF, GOC:TermGenie, GOC:mtg_cardiac_conduct_nov11, GOC:rl, GO_REF:0000059 Also known as: down regulation of Kir channel activity, down regulation of inward rectifier potassium channel activity, down-regulation of Kir channel activity, down-regulation of inward rectifier potassium channel activity, downregulation of Kir channel activity, downregulation of inward rectifier potassium channel activity, negative regulation of Kir channel activity, inhibition of Kir channel activity, inhibition of inward rectifier potassium channel activity Relationships: is a type of negative regulation of voltage-gated potassium channel activity [GO:1903817]; negatively regulates inward rectifier potassium channel activity [GO:0005242]